{
  "term_label": "COPII-coated ER to Golgi transport vesicle",
  "gene_symbol": "LMAN2L",
  "term_id": "GO:0030134",
  "gene": "UniProtKB:Q9H0V9",
  "gene_name": "VIP36-like protein"
}